{
  "gene": "UniProtKB:P37275",
  "term_label": "regulation of transcription by RNA polymerase II",
  "term_id": "GO:0006357",
  "gene_name": "Zinc finger E-box-binding homeobox 1",
  "gene_symbol": "ZEB1"
}